corticotropin hormone secreting cell development [GO:0060131] (BP) Sources: GOC:dph Relationships: is a type of GO:0048468; is part of corticotropin hormone secreting cell differentiation [GO:0060128] Definition: The process whose specific outcome is the progression of a corticotropic hormone secreting cell over time, from its formation to the mature structure. An corticotropic hormone secreting cell is a basophil cell of the anterior pituitary that produces corticotropin. Also known as: adrenocorticotrophic hormone secreting cell development, adrenocorticotropic hormone secreting cell development, corticotrope development, corticotroph development, corticotrophin hormone secreting cell development